regulation of calcitonin secretion [GO:1904362] (biological process) Subtypes: negative regulation of calcitonin secretion [GO:1904363], positive regulation of calcitonin secretion [GO:1904364] Definition: Any process that modulates the frequency, rate or extent of calcitonin secretion. Relationships: is a type of regulation of peptide hormone secretion [GO:0090276]; regulates GO:0036161 References: PMID:11278900 Sources: GOC:TermGenie, GO_REF:0000058